{
  "gene_symbol": "PARP8",
  "gene_name": "Protein mono-ADP-ribosyltransferase PARP8",
  "term_label": "endoplasmic reticulum unfolded protein response",
  "gene": "UniProtKB:Q8N3A8",
  "term_id": "GO:0030968"
}